{
  "gene_name": "Biliverdin reductase A",
  "gene": "UniProtKB:P53004",
  "gene_symbol": "BLVRA",
  "term_id": "UNKNOWN:0003",
  "term_label": "Unknown cellular component"
}